{
  "gene_symbol": "GDI2",
  "gene_name": "Rab GDP dissociation inhibitor beta",
  "term_id": "GO:0005093",
  "gene": "UniProtKB:P50395",
  "term_label": "Rab GDP-dissociation inhibitor activity"
}